{
  "term_label": "Unknown cellular component",
  "gene": "UniProtKB:Q12951",
  "gene_name": "Forkhead box protein I1",
  "gene_symbol": "FOXI1",
  "term_id": "UNKNOWN:0003"
}